bundle of His development [GO:0003166] (biological process) Also known as: atrioventricular bundle development Definition: The process whose specific outcome is the progression of the bundle of His over time, from its formation to the mature structure. The bundle of His is part of the His-Purkinje system that transmits signals from the AV node to the cardiac Purkinje fibers. Sources: GOC:mtg_heart Relationships: is a type of ventricular cardiac muscle tissue development [GO:0003229]; is part of GO:0003164